clathrin-sculpted gamma-aminobutyric acid transport vesicle lumen [GO:0061201] (cellular component) Relationships: is a type of cytoplasmic vesicle lumen [GO:0060205]; is part of GO:0061200 Also known as: clathrin sculpted GABA transport vesicle lumen, clathrin sculpted gamma-aminobutyric acid transport vesicle lumen Definition: The volume enclosed by the membrane of the clathrin-sculpted gamma-aminobutyric acid transport vesicle. Sources: GOC:dph